{
  "term_label": "Unknown cellular component",
  "term_id": "UNKNOWN:0003",
  "gene_name": "Protein PHTF2",
  "gene_symbol": "PHTF2",
  "gene": "UniProtKB:Q8N3S3"
}